{
  "gene_symbol": "CFLAR",
  "term_id": "GO:0030225",
  "gene_name": "CASP8 and FADD-like apoptosis regulator",
  "gene": "UniProtKB:O15519",
  "term_label": "macrophage differentiation"
}